{
  "gene_symbol": "SDF4",
  "term_id": "GO:0005509",
  "gene": "UniProtKB:Q9BRK5",
  "gene_name": "45 kDa calcium-binding protein",
  "term_label": "calcium ion binding"
}